{
  "gene": "UniProtKB:Q5EE01",
  "term_label": "Unknown molecular function",
  "gene_name": "Centromere protein W",
  "gene_symbol": "CENPW",
  "term_id": "UNKNOWN:0001"
}